{
  "gene_symbol": "RFC3",
  "gene_name": "Replication factor C subunit 3",
  "term_label": "DNA clamp loader activity",
  "term_id": "GO:0003689",
  "gene": "UniProtKB:P40938"
}